{
  "gene_symbol": "RAX2",
  "gene": "UniProtKB:Q96IS3",
  "term_label": "DNA-binding transcription factor activity, RNA polymerase II-specific",
  "gene_name": "Retina and anterior neural fold homeobox protein 2",
  "term_id": "GO:0000981"
}